{
  "gene_name": "Envoplakin-like protein",
  "gene_symbol": "EVPLL",
  "term_id": "UNKNOWN:0001",
  "term_label": "Unknown molecular function",
  "gene": "UniProtKB:A8MZ36"
}